recognition of pollen [GO:0048544] (biological process) Definition: A cell recognition process in which pollen is recognized and either accepted or rejected by cells in the stigma. Also known as: pollen recognition, recognition or rejection of self pollen, self incompatibility Subtypes: rejection of self pollen [GO:0060320], acceptance of pollen [GO:0060321], rejection of pollen from other species [GO:1990109] Relationships: is a type of GO:0008037 Sources: GOC:dph, GOC:pj, GOC:tb